Tle3-Aes complex [GO:0070722] (cellular component) Definition: A transcriptional repressor complex that consists of a heterodimer of the proteins Tle3 (also known as Grg3b) and Aes (Grg5), which are homologs of the Drosophila groucho gene product. References: PMID:8955148 Sources: GOC:mah Also known as: Grg3b-Grg5 complex Relationships: is a type of GO:0090571